{
  "term_label": "extracellular region",
  "term_id": "GO:0005576",
  "gene": "UniProtKB:Q9BQI4",
  "gene_symbol": "CCDC3",
  "gene_name": "Coiled-coil domain-containing protein 3"
}